aster [GO:0005818] (cellular component) Definition: An array of microtubules emanating from a spindle pole MTOC that do not connect to kinetochores. Subtypes: GO:0032117 Sources: GOC:clt Relationships: is a type of intracellular membraneless organelle [GO:0043232]; is a type of supramolecular complex [GO:0099080]; is part of spindle [GO:0005819]